root radial pattern formation [GO:0090057] (biological process) Definition: The radial pattern formation process that results in the formation of the different tissues of the root around its radial axis. Relationships: is a type of radial pattern formation [GO:0009956]; is part of root development [GO:0048364] Sources: GOC:dph, GOC:sdb_2009, GOC:tb